{
  "gene_symbol": "CCNI2",
  "gene_name": "Cyclin-I2",
  "gene": "UniProtKB:Q6ZMN8",
  "term_label": "G1/S transition of mitotic cell cycle",
  "term_id": "GO:0000082"
}